p-cumate biosynthetic process [GO:1901783] (biological process) Definition: The chemical reactions and pathways resulting in the formation of p-cumate. Also known as: p-cumate anabolism, p-cumate biosynthesis, p-cumate formation, p-cumate synthesis References: PMID:8631713 Sources: GOC:TermGenie, GOC:yaf Relationships: is a type of benzene-containing compound metabolic process [GO:0042537]; is_a monocarboxylic acid biosynthetic process [GO:0072330]